{
  "gene": "UniProtKB:P27469",
  "term_label": "mitochondrion",
  "gene_symbol": "G0S2",
  "gene_name": "G0_G1 switch protein 2",
  "term_id": "GO:0005739"
}